regulation of anatomical structure size [GO:0090066] (BP) Subtypes: GO:0032535, regulation of tube size [GO:0035150], regulation of kidney size [GO:0035564], regulation of imaginal disc-derived wing size [GO:0044719], regulation of thalamus size [GO:0090067], GO:1903814, regulation of lymphatic vessel size [GO:1990186] Sources: GOC:dph, GOC:tb Definition: Any process that modulates the size of an anatomical structure. Relationships: is a type of GO:0065008